regulation of kojic acid biosynthetic process [GO:1900394] (biological process) Also known as: regulation of 5-hydroxy-2-(hydroxymethyl)-4H-pyran-4-one anabolism, regulation of 5-hydroxy-2-(hydroxymethyl)-4H-pyran-4-one biosynthesis, regulation of 5-hydroxy-2-(hydroxymethyl)-4H-pyran-4-one biosynthetic process, regulation of 5-hydroxy-2-(hydroxymethyl)-4H-pyran-4-one formation, regulation of 5-hydroxy-2-(hydroxymethyl)-4H-pyran-4-one synthesis, regulation of kojic acid anabolism, regulation of kojic acid biosynthesis, regulation of kojic acid formation, regulation of kojic acid synthesis, regulation of C6H6O4 anabolism, regulation of C6H6O4 biosynthesis, regulation of C6H6O4 biosynthetic process, regulation of C6H6O4 formation, regulation of C6H6O4 synthesis Sources: GOC:TermGenie, GOC:di Definition: Any process that modulates the frequency, rate or extent of kojic acid biosynthetic process. Subtypes: negative regulation of kojic acid biosynthetic process [GO:1900395], positive regulation of kojic acid biosynthetic process [GO:1900396] Relationships: is a type of GO:0010566; is a type of regulation of alcohol biosynthetic process [GO:1902930]; regulates kojic acid biosynthetic process [GO:2001317]